{
  "gene_symbol": "HYAL4",
  "gene": "UniProtKB:Q2M3T9",
  "term_id": "GO:0004415",
  "term_label": "hyalurononglucosaminidase activity",
  "gene_name": "Hyaluronidase-4"
}